amnioserosa formation [GO:0007378] (biological process) Sources: ISBN:0879694238 Definition: Formation of the amnioserosa, an epithelium that occupies a hole in the embryonic dorsal epidermis. This occurs by the transformation of a narrow strip of cells at the dorsal midline of the blastoderm from columnar to squamous cells, accompanied by a lateral shift. Relationships: is a type of GO:0048646; is part of gastrulation involving germ band extension [GO:0010004]